{
  "gene_symbol": "SERTAD1",
  "gene": "UniProtKB:Q9UHV2",
  "term_label": "Unknown biological process",
  "term_id": "UNKNOWN:0002",
  "gene_name": "SERTA domain-containing protein 1"
}